{
  "term_id": "GO:0006435",
  "gene_name": "Threonine--tRNA ligase 2, cytoplasmic",
  "gene_symbol": "TARS3",
  "gene": "UniProtKB:A2RTX5",
  "term_label": "threonyl-tRNA aminoacylation"
}